{
  "term_label": "intracellular iron ion homeostasis",
  "gene_symbol": "GLRX3",
  "term_id": "GO:0006879",
  "gene_name": "Glutaredoxin-3",
  "gene": "UniProtKB:O76003"
}